{
  "gene_symbol": "KIFBP",
  "term_id": "UNKNOWN:0001",
  "gene_name": "KIF-binding protein",
  "term_label": "Unknown molecular function",
  "gene": "UniProtKB:Q96EK5"
}